{
  "term_label": "cytosol",
  "gene_symbol": "UBQLNL",
  "gene": "UniProtKB:Q8IYU4",
  "term_id": "GO:0005829",
  "gene_name": "Ubiquilin-like protein"
}